{
  "gene_name": "CDK5 regulatory subunit-associated protein 3",
  "gene": "UniProtKB:Q96JB5",
  "gene_symbol": "CDK5RAP3",
  "term_id": "GO:0012505",
  "term_label": "endomembrane system"
}